{
  "gene": "UniProtKB:P07478",
  "term_label": "proteolysis",
  "gene_symbol": "PRSS2",
  "gene_name": "Trypsin-2",
  "term_id": "GO:0006508"
}